{
  "gene_symbol": "TBC1D3E",
  "gene": "UniProtKB:A0A087X179",
  "gene_name": "TBC1 domain family member 3E",
  "term_id": "UNKNOWN:0002",
  "term_label": "Unknown biological process"
}